{
  "gene_name": "Protein FAM135A",
  "gene": "UniProtKB:Q9P2D6",
  "term_label": "lipid metabolic process",
  "term_id": "GO:0006629",
  "gene_symbol": "FAM135A"
}